unsaturated fatty acid biosynthetic process [GO:0006636] (biological process) Definition: The chemical reactions and pathways resulting in the formation of an unsaturated fatty acid, any fatty acid containing one or more double bonds between carbon atoms. Sources: GOC:mah, MetaCyc:PWY-762, MetaCyc:PWY-782 Also known as: unsaturated fatty acid anabolism, unsaturated fatty acid biosynthesis, unsaturated fatty acid formation, unsaturated fatty acid synthesis, polyunsaturated fatty acid biosynthesis, fatty acid desaturation Relationships: is a type of fatty acid biosynthetic process [GO:0006633]; is a type of unsaturated fatty acid metabolic process [GO:0033559] Subtypes: prostanoid biosynthetic process [GO:0046457], (R)-2-hydroxy-alpha-linolenic acid biosynthetic process [GO:1902609], GO:2001303, GO:2001306 Regulation: regulated by regulation of unsaturated fatty acid biosynthetic process [GO:2001279]; positively regulated by positive regulation of unsaturated fatty acid biosynthetic process [GO:2001280]